{
  "term_id": "GO:0006368",
  "gene_symbol": "SUPT6H",
  "gene": "UniProtKB:Q7KZ85",
  "term_label": "transcription elongation by RNA polymerase II",
  "gene_name": "Transcription elongation factor SPT6"
}